negative regulation of helicase activity [GO:0051097] (biological process) Sources: GOC:ai Definition: Any process that stops or reduces the activity of a helicase. Also known as: down regulation of helicase activity, down-regulation of helicase activity, downregulation of helicase activity, inhibition of helicase activity Relationships: is a type of negative regulation of ATP-dependent activity [GO:0032780]; is a type of negative regulation of catalytic activity [GO:0043086]; RO_0002212 helicase activity [GO:0004386]